{
  "gene": "UniProtKB:Q8NA72",
  "gene_name": "Centrosomal protein POC5",
  "gene_symbol": "POC5",
  "term_label": "Unknown molecular function",
  "term_id": "UNKNOWN:0001"
}